{
  "gene_symbol": "AZIN1",
  "gene": "UniProtKB:O14977",
  "term_label": "cytoplasm",
  "gene_name": "Antizyme inhibitor 1",
  "term_id": "GO:0005737"
}